{
  "gene_symbol": "SLC9B2",
  "term_id": "UNKNOWN:0002",
  "term_label": "Unknown biological process",
  "gene": "UniProtKB:Q86UD5",
  "gene_name": "Sodium_hydrogen exchanger 9B2"
}